{
  "term_label": "sialic acid transmembrane transporter activity",
  "term_id": "GO:0015136",
  "gene": "UniProtKB:Q9NRA2",
  "gene_name": "Sialin",
  "gene_symbol": "SLC17A5"
}